{
  "term_id": "GO:0043161",
  "gene_name": "Phospholipase A-2-activating protein",
  "gene_symbol": "PLAA",
  "gene": "UniProtKB:Q9Y263",
  "term_label": "proteasome-mediated ubiquitin-dependent protein catabolic process"
}